{
  "gene_name": "Protein O-mannosyl-transferase TMTC4",
  "gene_symbol": "TMTC4",
  "gene": "UniProtKB:Q5T4D3",
  "term_label": "protein O-linked glycosylation via mannose",
  "term_id": "GO:0035269"
}